inflammasome-mediated signaling pathway [GO:0141084] (biological process) Definition: An intracellular signal transduction pathway that starts with a ligand binding to a pattern recognition receptor (PRR), assembly of the inflammasome complex, leading to the activation of CASP1 and inducing an inflammatory response. In some cases, inflammasome-mediated signal transduction can lead to programmed cell death, such as pyroptosis. Regulation: regulated by regulation of inflammasome-mediated signaling pathway [GO:0141085]; RO_0002212 by negative regulation of inflammasome-mediated signaling pathway [GO:0141086]; positively regulated by positive regulation of inflammasome-mediated signaling pathway [GO:0141087] Also known as: inflammasome-mediated signal transduction References: PMID:35883561 Relationships: is a type of cytoplasmic pattern recognition receptor signaling pathway [GO:0002753]; BFO_0000050 GO:0006954